{
  "term_label": "canonical glycolysis",
  "gene": "UniProtKB:P15259",
  "gene_symbol": "PGAM2",
  "term_id": "GO:0061621",
  "gene_name": "Phosphoglycerate mutase 2"
}